negative regulation of maintenance of mitotic sister chromatid cohesion, centromeric [GO:2000719] (BP) Sources: GOC:mah Definition: Any process that stops, prevents or reduces the frequency, rate or extent of maintenance of mitotic sister chromatid cohesion in the centromeric region. Relationships: is_a negative regulation of maintenance of mitotic sister chromatid cohesion [GO:0034183]; is a type of regulation of maintenance of mitotic sister chromatid cohesion, centromeric [GO:2000718]; negatively regulates GO:0071960 Also known as: negative regulation of maintenance of centromeric mitotic sister chromatin cohesion, negative regulation of maintenance of mitotic sister chromatin cohesion at centromere, negative regulation of maintenance of sister chromatin cohesion at centromere at mitosis